4-methyloxaloacetate esterase activity [GO:0047583] (molecular function) Also known as: oxaloacetate-4-methyl-ester oxaloacetohydrolase activity Sources: EC:3.1.1.44, RHEA:10564 Relationships: is a type of carboxylic ester hydrolase activity [GO:0052689] Definition: Catalysis of the reaction: 4-methoxy-2,4-dioxobutanoate + H2O = H+ + methanol + oxaloacetate.